{
  "gene_name": "Interferon alpha-2",
  "term_id": "GO:0002286",
  "gene_symbol": "IFNA2",
  "term_label": "T cell activation involved in immune response",
  "gene": "UniProtKB:P01563"
}